{
  "term_label": "extracellular matrix",
  "gene_name": "Collagen alpha-4(IV) chain",
  "gene_symbol": "COL4A4",
  "gene": "UniProtKB:P53420",
  "term_id": "GO:0031012"
}